sphinganine metabolic process [GO:0006667] (biological process) References: PMID:29165427 Relationships: is a type of diol metabolic process [GO:0034311]; is a type of sphingoid metabolic process [GO:0046519] Subtypes: sphinganine biosynthetic process [GO:0046511] Definition: The chemical reactions and pathways involving sphinganine, D-erythro-2-amino-1,3-octadecanediol. Also known as: dihydrosphingosine metabolic process, dihydrosphingosine metabolism, sphinganine metabolism